{
  "term_id": "GO:0043005",
  "term_label": "neuron projection",
  "gene": "UniProtKB:P48145",
  "gene_symbol": "NPBWR1",
  "gene_name": "Neuropeptides B_W receptor type 1"
}